{
  "term_id": "GO:0005730",
  "gene_name": "RNA cytidine acetyltransferase",
  "gene": "UniProtKB:Q9H0A0",
  "term_label": "nucleolus",
  "gene_symbol": "NAT10"
}